positive regulation of glycine import across plasma membrane [GO:1900925] (biological process) Definition: Any process that activates or increases the frequency, rate or extent of glycine import. Sources: GOC:TermGenie Also known as: positive regulation of glycine import, up regulation of glycine import, up-regulation of glycine import, upregulation of glycine import, activation of glycine import Relationships: is a type of positive regulation of organic acid transport [GO:0032892]; is a type of positive regulation of transmembrane transport [GO:0034764]; is_a GO:0051957; is a type of regulation of glycine import across plasma membrane [GO:1900923]; positively regulates glycine import across plasma membrane [GO:1903804]